{
  "term_id": "UNKNOWN:0003",
  "term_label": "Unknown cellular component",
  "gene_symbol": "S100Z",
  "gene": "UniProtKB:Q8WXG8",
  "gene_name": "Protein S100-Z"
}